{
  "gene": "UniProtKB:Q8NFW1",
  "term_id": "GO:0005604",
  "gene_name": "Collagen alpha-1(XXII) chain",
  "gene_symbol": "COL22A1",
  "term_label": "basement membrane"
}